V1B vasopressin receptor binding [GO:0031895] (molecular function) Also known as: V1B vasopressin receptor ligand Relationships: is a type of vasopressin receptor binding [GO:0031893] Sources: GOC:mah, GOC:nln Definition: Binding to a V1B vasopressin receptor.